plasma membrane copper ion transport [GO:0015679] (biological process) Sources: GOC:ai Subtypes: copper ion import across plasma membrane [GO:0098705] Relationships: is a type of copper ion transmembrane transport [GO:0035434] Also known as: plasma membrane copper transport Definition: The directed movement of copper ions across the plasma membrane.